{
  "gene_name": "NBAS subunit of NRZ tethering complex",
  "term_label": "retrograde vesicle-mediated transport, Golgi to endoplasmic reticulum",
  "term_id": "GO:0006890",
  "gene_symbol": "NBAS",
  "gene": "UniProtKB:A2RRP1"
}